{
  "gene_symbol": "RETN",
  "term_id": "GO:0005615",
  "gene": "UniProtKB:Q9HD89",
  "gene_name": "Resistin",
  "term_label": "extracellular space"
}